{
  "gene_symbol": "PRKAB2",
  "gene_name": "5'-AMP-activated protein kinase subunit beta-2",
  "term_id": "GO:0031588",
  "gene": "UniProtKB:O43741",
  "term_label": "nucleotide-activated protein kinase complex"
}